{
  "term_label": "inner acrosomal membrane",
  "gene": "UniProtKB:Q8WZ59",
  "gene_name": "Transmembrane protein 190",
  "term_id": "GO:0002079",
  "gene_symbol": "TMEM190"
}